tropism [GO:0009606] (biological process) Definition: The movement of an organism, or part of an organism, in response to an external source of stimulus, usually toward or away from it. Sources: GOC:curators, ISBN:0877795088 Relationships: is a type of response to external stimulus [GO:0009605] Subtypes: gravitropism [GO:0009630], phototropism [GO:0009638], thigmotropism [GO:0009652], hydrotropism [GO:0010274], chemotropism [GO:0043577], halotropism [GO:0170002]